inner mucus layer [GO:0070702] (cellular component) References: PMID:18806221, PMID:19432394 Sources: GOC:mah, GOC:mm2 Definition: The inner of two mucus layers secreted by epithelial cells in the colon; the inner mucus layer is firmly attached to the epithelium, is densely packed with a compact stratified appearance and is devoid of bacteria. Relationships: is a type of mucus layer [GO:0070701]